{
  "term_label": "extracellular space",
  "gene": "UniProtKB:Q6UVY6",
  "gene_name": "DBH-like monooxygenase protein 1",
  "term_id": "GO:0005615",
  "gene_symbol": "MOXD1"
}